{
  "term_id": "GO:0003729",
  "term_label": "mRNA binding",
  "gene_symbol": "DDX4",
  "gene": "UniProtKB:Q9NQI0",
  "gene_name": "Probable ATP-dependent RNA helicase DDX4"
}